regulation of hormone secretion [GO:0046883] (biological process) Relationships: is a type of regulation of cell communication [GO:0010646]; is_a regulation of hormone levels [GO:0010817]; is a type of regulation of signaling [GO:0023051]; is a type of regulation of secretion by cell [GO:1903530]; regulates hormone secretion [GO:0046879] Definition: Any process that modulates the frequency, rate or extent of the regulated release of a hormone from a cell. Sources: GOC:ai Subtypes: regulation of juvenile hormone secretion [GO:0007558], GO:0032276, GO:0032335, regulation of inhibin secretion [GO:0032338], GO:0046887, negative regulation of hormone secretion [GO:0046888], regulation of adiponectin secretion [GO:0070163], regulation of peptide hormone secretion [GO:0090276], GO:1903593, regulation of parathyroid hormone secretion [GO:2000828], regulation of steroid hormone secretion [GO:2000831], regulation of androstenedione secretion [GO:2000837], GO:2000840, regulation of testosterone secretion [GO:2000843]